{
  "gene_name": "Leucine-rich repeat protein SHOC-2",
  "term_label": "positive regulation of Ras protein signal transduction",
  "gene_symbol": "SHOC2",
  "gene": "UniProtKB:Q9UQ13",
  "term_id": "GO:0046579"
}